{
  "gene_name": "Signal transducer and activator of transcription 4",
  "term_label": "nucleus",
  "gene": "UniProtKB:Q14765",
  "term_id": "GO:0005634",
  "gene_symbol": "STAT4"
}